3-oxoadipate CoA-transferase activity [GO:0047569] (molecular function) Definition: Catalysis of the reaction: succinyl-CoA + 3-oxoadipate = succinate + 3-oxoadipyl-CoA. Also known as: 3-oxoadipate coenzyme A-transferase activity, 3-oxoadipate succinyl-CoA transferase activity, beta-ketoadipate:succinyl-CoA transferase activity, succinyl-CoA:3-oxoadipate CoA-transferase activity Sources: EC:2.8.3.6, MetaCyc:3-OXOADIPATE-COA-TRANSFERASE-RXN Relationships: is a type of CoA-transferase activity [GO:0008410]